{
  "term_id": "GO:1905515",
  "gene_name": "Protein fantom",
  "gene": "UniProtKB:Q68CZ1",
  "gene_symbol": "RPGRIP1L",
  "term_label": "non-motile cilium assembly"
}